{
  "gene_symbol": "CLEC9A",
  "gene": "UniProtKB:Q6UXN8",
  "gene_name": "C-type lectin domain family 9 member A",
  "term_id": "UNKNOWN:0001",
  "term_label": "Unknown molecular function"
}